{
  "term_label": "kinesin complex",
  "gene": "UniProtKB:Q8N4N8",
  "gene_symbol": "KIF2B",
  "term_id": "GO:0005871",
  "gene_name": "Kinesin-like protein KIF2B"
}